{
  "gene_symbol": "LY96",
  "term_label": "lipopolysaccharide receptor complex",
  "term_id": "GO:0046696",
  "gene_name": "Lymphocyte antigen 96",
  "gene": "UniProtKB:Q9Y6Y9"
}